mesenchymal stem cell migration [GO:1905319] (biological process) Definition: The orderly movement of a mesenchymal stem cell from one site to another. References: PMID:24924806, PMID:25181476 Sources: GOC:TermGenie, GO_REF:0000091 Relationships: is a type of GO:0016477 Regulation: regulated by regulation of mesenchymal stem cell migration [GO:1905320]; negatively regulated by negative regulation of mesenchymal stem cell migration [GO:1905321]; positively regulated by GO:1905322